{
  "term_label": "proteasome-mediated ubiquitin-dependent protein catabolic process",
  "gene": "UniProtKB:Q96MT1",
  "gene_symbol": "RNF145",
  "gene_name": "RING finger protein 145",
  "term_id": "GO:0043161"
}